{
  "term_label": "chromatin",
  "gene_symbol": "TBX21",
  "term_id": "GO:0000785",
  "gene_name": "T-box transcription factor TBX21",
  "gene": "UniProtKB:Q9UL17"
}